{
  "gene": "UniProtKB:A0A087WWU0",
  "term_label": "Unknown molecular function",
  "term_id": "UNKNOWN:0001",
  "gene_name": "Uncharacterized protein (Fragment)",
  "gene_symbol": "A0A087WWU0"
}